{
  "term_label": "RNA endonuclease activity",
  "gene_symbol": "AGO3",
  "gene": "UniProtKB:Q9H9G7",
  "term_id": "GO:0004521",
  "gene_name": "Protein argonaute-3"
}